{
  "gene_name": "Probable non-functional immunoglobulin heavy variable 3-38",
  "gene_symbol": "IGHV3-38",
  "term_id": "UNKNOWN:0003",
  "term_label": "Unknown cellular component",
  "gene": "UniProtKB:A0A0C4DH36"
}